{
  "gene": "UniProtKB:Q7Z3H4",
  "gene_name": "Sterile alpha motif domain-containing protein 7",
  "term_label": "histone binding",
  "gene_symbol": "SAMD7",
  "term_id": "GO:0042393"
}